{
  "gene_name": "Allograft inflammatory factor 1",
  "term_id": "GO:0051017",
  "gene": "UniProtKB:P55008",
  "gene_symbol": "AIF1",
  "term_label": "actin filament bundle assembly"
}